{
  "gene_name": "Bargin",
  "gene": "UniProtKB:Q6ZT62",
  "term_id": "GO:0005829",
  "term_label": "cytosol",
  "gene_symbol": "BARGIN"
}